{
  "term_label": "Unknown cellular component",
  "gene": "UniProtKB:Q9NV12",
  "gene_symbol": "TMEM140",
  "gene_name": "Transmembrane protein 140",
  "term_id": "UNKNOWN:0003"
}